{
  "gene_name": "Tumor necrosis factor receptor superfamily member 11A",
  "gene_symbol": "TNFRSF11A",
  "term_label": "multinuclear osteoclast differentiation",
  "term_id": "GO:0072674",
  "gene": "UniProtKB:Q9Y6Q6"
}